{
  "term_id": "GO:0005249",
  "gene_symbol": "LRRC38",
  "gene_name": "Leucine-rich repeat-containing protein 38",
  "gene": "UniProtKB:Q5VT99",
  "term_label": "voltage-gated potassium channel activity"
}